{
  "gene_name": "Alpha-ketoglutarate-dependent dioxygenase alkB homolog 4",
  "term_id": "GO:0016706",
  "gene_symbol": "ALKBH4",
  "gene": "UniProtKB:Q9NXW9",
  "term_label": "2-oxoglutarate-dependent dioxygenase activity"
}